positive regulation of sporangium germination [GO:0075224] (biological process) Relationships: is_a regulation of sporangium germination [GO:0075223]; is a type of positive regulation of sporangium development [GO:0075311]; positively regulates sporangium germination [GO:0075222] Also known as: positive regulation of sporangium germination on or near host Definition: Any process that activates, maintains or increases the frequency, rate or extent of sporangium germination. Sources: GOC:pamgo_curators